cytoplasmic lattice [GO:0140095] (cellular component) Definition: Fibrous structures of the mammalian ooplasm that store ribosomes and maternal proteins in insoluble form to prevent their degradation, activation and nuclear transfer. Relationships: is a type of intracellular membraneless organelle [GO:0043232]; is part of ooplasm [GO:1990917] References: PMID:37922900, PMID:38955588